{
  "gene": "UniProtKB:P15848",
  "term_label": "Unknown biological process",
  "term_id": "UNKNOWN:0002",
  "gene_symbol": "ARSB",
  "gene_name": "Arylsulfatase B"
}